{
  "term_label": "retrograde vesicle-mediated transport, Golgi to endoplasmic reticulum",
  "term_id": "GO:0006890",
  "gene": "UniProtKB:Q9NRW1",
  "gene_name": "Ras-related protein Rab-6B",
  "gene_symbol": "RAB6B"
}